{
  "term_label": "nucleus",
  "gene_name": "Heterogeneous nuclear ribonucleoprotein R",
  "term_id": "GO:0005634",
  "gene_symbol": "HNRNPR",
  "gene": "UniProtKB:O43390"
}